{
  "gene": "UniProtKB:P0DMU2",
  "term_id": "GO:0007608",
  "gene_name": "Putative olfactory receptor 8G3 pseudogene",
  "gene_symbol": "OR8G3",
  "term_label": "sensory perception of smell"
}